{
  "gene_symbol": "GRXCR1",
  "gene_name": "Glutaredoxin domain-containing cysteine-rich protein 1",
  "term_id": "GO:0060122",
  "gene": "UniProtKB:A8MXD5",
  "term_label": "inner ear receptor cell stereocilium organization"
}